{
  "term_label": "DNA-binding transcription factor activity, RNA polymerase II-specific",
  "gene": "UniProtKB:Q6IV72",
  "term_id": "GO:0000981",
  "gene_symbol": "ZNF425",
  "gene_name": "Zinc finger protein 425"
}